gluconate dehydrogenase activity [GO:0008875] (molecular function) Relationships: is a type of GO:0016616 Subtypes: gluconate 2-dehydrogenase activity [GO:0008873], gluconate 5-dehydrogenase activity [GO:0008874], gluconate 2-dehydrogenase (acceptor) activity [GO:0033717] Sources: GOC:curators Definition: Catalysis of the reaction: D-gluconate + NADP+ = dehydro-D-gluconate + NADPH + H+.